{
  "gene_symbol": "LIMK1",
  "term_id": "GO:0051496",
  "gene_name": "LIM domain kinase 1",
  "term_label": "positive regulation of stress fiber assembly",
  "gene": "UniProtKB:P53667"
}